{
  "term_id": "UNKNOWN:0002",
  "term_label": "Unknown biological process",
  "gene": "UniProtKB:Q6ZSA7",
  "gene_symbol": "LRRC55",
  "gene_name": "Leucine-rich repeat-containing protein 55"
}